{
  "gene": "UniProtKB:A6PVC2",
  "gene_symbol": "TTLL8",
  "term_label": "axoneme assembly",
  "term_id": "GO:0035082",
  "gene_name": "Protein monoglycylase TTLL8"
}